cyanogenic glycoside catabolic process [GO:0042342] (biological process) Relationships: is a type of glycoside catabolic process [GO:0016139]; is a type of nitrile catabolic process [GO:0050899] Definition: The chemical reactions and pathways resulting in the breakdown of cyanogenic glycosides, any glycoside containing a cyano group that is released as hydrocyanic acid on acid hydrolysis; such compounds occur in the kernels of various fruits. Also known as: cyanogenic glycoside breakdown, cyanogenic glycoside catabolism, cyanogenic glycoside degradation Sources: ISBN:0198506732